{
  "gene_symbol": "CD74",
  "term_id": "GO:1902166",
  "gene": "UniProtKB:P04233",
  "term_label": "negative regulation of intrinsic apoptotic signaling pathway in response to DNA damage by p53 class mediator",
  "gene_name": "HLA class II histocompatibility antigen gamma chain"
}